{
  "term_id": "UNKNOWN:0001",
  "term_label": "Unknown molecular function",
  "gene_symbol": "CLPTM1L",
  "gene_name": "Lipid scramblase CLPTM1L",
  "gene": "UniProtKB:Q96KA5"
}